{
  "term_label": "t-UTP complex",
  "gene_symbol": "UTP4",
  "gene": "UniProtKB:Q969X6",
  "gene_name": "U3 small nucleolar RNA-associated protein 4 homolog",
  "term_id": "GO:0034455"
}